{
  "gene": "UniProtKB:P07205",
  "term_label": "cytosol",
  "term_id": "GO:0005829",
  "gene_symbol": "PGK2",
  "gene_name": "Phosphoglycerate kinase 2"
}